{
  "gene_name": "Zinc finger protein 266",
  "gene_symbol": "ZNF266",
  "term_id": "GO:0000981",
  "gene": "UniProtKB:Q14584",
  "term_label": "DNA-binding transcription factor activity, RNA polymerase II-specific"
}